{
  "term_label": "Unknown biological process",
  "term_id": "UNKNOWN:0002",
  "gene": "UniProtKB:Q8IVE0",
  "gene_name": "Putative ciliary rootlet coiled-coil protein-like 2 protein",
  "gene_symbol": "CROCCP3"
}